{
  "term_label": "mitotic spindle assembly",
  "term_id": "GO:0090307",
  "gene_name": "BRCA1-A complex subunit Abraxas 1",
  "gene": "UniProtKB:Q6UWZ7",
  "gene_symbol": "ABRAXAS1"
}